{
  "term_label": "RNA helicase activity",
  "term_id": "GO:0003724",
  "gene_symbol": "DHX36",
  "gene_name": "ATP-dependent DNA_RNA helicase DHX36",
  "gene": "UniProtKB:Q9H2U1"
}